{
  "gene": "UniProtKB:Q63HQ0",
  "gene_symbol": "AP1AR",
  "term_label": "vesicle targeting, trans-Golgi to endosome",
  "gene_name": "AP-1 complex-associated regulatory protein",
  "term_id": "GO:0048203"
}